{
  "term_label": "plasma membrane",
  "gene": "UniProtKB:B6A8C7",
  "gene_name": "T-cell-interacting, activating receptor on myeloid cells protein 1",
  "term_id": "GO:0005886",
  "gene_symbol": "TARM1"
}